voltage-gated sodium channel activity involved in Purkinje myocyte action potential [GO:0086062] (molecular function) Definition: Enables the transmembrane transfer of a sodium ion by a voltage-gated channel through the plasma membrane of a Purkinje myocyte contributing to the depolarization phase of an action potential. A voltage-gated channel is a channel whose open state is dependent on the voltage across the membrane in which it is embedded. Sources: GOC:BHF, GOC:mtg_cardiac_conduct_nov11 Relationships: is_a voltage-gated sodium channel activity involved in cardiac muscle cell action potential [GO:0086006]; is part of membrane depolarization during Purkinje myocyte cell action potential [GO:0086047]